{
  "gene_name": "Mitochondrial fission 1 protein",
  "gene_symbol": "FIS1",
  "term_label": "mitochondrial fission",
  "gene": "UniProtKB:Q9Y3D6",
  "term_id": "GO:0000266"
}